toll-like receptor 3 signaling pathway [GO:0034138] (biological process) Regulation: RO_0002211 by GO:0034139; negatively regulated by negative regulation of toll-like receptor 3 signaling pathway [GO:0034140]; positively regulated by positive regulation of toll-like receptor 3 signaling pathway [GO:0034141] Also known as: TLR3 signaling pathway, toll-like receptor 3 signalling pathway Definition: The series of molecular signals initiated by a ligand binding to the endolysosomal toll-like receptor 3. Relationships: is a type of endolysosomal toll-like receptor signaling pathway [GO:0140894] References: PMID:16551253, PMID:17328678 Sources: GOC:add